{
  "gene_symbol": "SHTN1",
  "gene": "UniProtKB:A0MZ66",
  "term_label": "Unknown molecular function",
  "term_id": "UNKNOWN:0001",
  "gene_name": "Shootin-1"
}